invasive growth in response to abiotic stimulus [GO:0097318] (biological process) Relationships: is a type of response to abiotic stimulus [GO:0009628]; is_a invasive filamentous growth [GO:0036267] References: PMID:18679170 Sources: GOC:di Definition: The growth of colonies in filamentous chains of cells as a result of a abiotic stimulus. An example of this process is found in Candida albicans.